establishment of Sertoli cell barrier [GO:0097368] (biological process) References: PMID:19509333 Sources: GOC:sl, Wikipedia:Blood-testis_barrier Regulation: regulated by GO:1904444; negatively regulated by negative regulation of establishment of Sertoli cell barrier [GO:1904445]; positively regulated by GO:1904446 Relationships: is a type of GO:0060009 Also known as: establishment of BTB, establishment of SCB, establishment of blood-testis barrier Definition: Establishment of a structure near the basement membrane in adjacent Sertoli cells of the seminiferous epithelium for maintaining spermatogenesis. The structure consists of tight junctions, basal ectoplasmic specializations, and desmosome-like junctions.